{
  "term_id": "GO:0017159",
  "gene_name": "Pantetheine hydrolase VNN2",
  "gene_symbol": "VNN2",
  "term_label": "pantetheine hydrolase activity",
  "gene": "UniProtKB:O95498"
}